{
  "term_label": "Unknown molecular function",
  "gene_symbol": "PREPL",
  "term_id": "UNKNOWN:0001",
  "gene_name": "Prolyl endopeptidase-like",
  "gene": "UniProtKB:Q4J6C6"
}